{
  "gene": "UniProtKB:Q5VZE5",
  "term_label": "negative regulation of apoptotic process",
  "gene_name": "N-alpha-acetyltransferase 35, NatC auxiliary subunit",
  "term_id": "GO:0043066",
  "gene_symbol": "NAA35"
}